{
  "term_id": "UNKNOWN:0003",
  "gene_name": "CCAAT_enhancer-binding protein delta",
  "gene_symbol": "CEBPD",
  "gene": "UniProtKB:P49716",
  "term_label": "Unknown cellular component"
}